{
  "term_id": "GO:0005813",
  "gene": "UniProtKB:Q99996",
  "gene_symbol": "AKAP9",
  "term_label": "centrosome",
  "gene_name": "A-kinase anchor protein 9"
}